negative regulation of striated muscle cell differentiation [GO:0051154] (biological process) Relationships: is a type of GO:0051148; is a type of regulation of striated muscle cell differentiation [GO:0051153]; negatively regulates striated muscle cell differentiation [GO:0051146] Also known as: down regulation of striated muscle cell differentiation, down-regulation of striated muscle cell differentiation, downregulation of striated muscle cell differentiation, inhibition of striated muscle cell differentiation Definition: Any process that stops, prevents, or reduces the frequency, rate or extent of striated muscle cell differentiation. Subtypes: negative regulation of myotube differentiation [GO:0010832], negative regulation of skeletal muscle fiber development [GO:0048744], negative regulation of cardiac muscle fiber development [GO:0055019], negative regulation of cell growth involved in cardiac muscle cell development [GO:0061052], GO:2000726 Sources: CL:0000737, GOC:ai